hormone-mediated apoptotic signaling pathway [GO:0008628] (biological process) Also known as: apoptotic signaling pathway in response to hormone, induction of apoptosis by hormones Note: This term is placed under GO:0097190 apoptotic signaling pathway, rather than under one of its more specific children terms, to cover for the variety of apoptosis signaling mechanisms that different hormones may use. Sources: GOC:bf, GOC:mtg_apoptosis Relationships: is a type of GO:0009755; is a type of apoptotic signaling pathway [GO:0097190] Definition: The series of molecular signals mediated by the detection of a hormone, and which triggers the apoptotic signaling pathway in a cell. The pathway starts with reception of a hormone signal, and ends when the execution phase of apoptosis is triggered.